branched-dextran exo-1,2-alpha-glucosidase activity [GO:0033933] (molecular function) Relationships: is a type of alpha-glucosidase activity [GO:0090599] Also known as: 1,2-alpha-D-glucosyl-branched-dextran 2-glucohydrolase activity, dextran 1,2-alpha-glucosidase activity, dextran alpha-1,2 debranching enzyme Definition: Catalysis of the hydrolysis of (1->2)-alpha-D-glucosidic linkages at the branch points of dextrans and related polysaccharides, producing free D-glucose. Sources: EC:3.2.1.115